{
  "term_id": "GO:0048268",
  "gene": "UniProtKB:O00291",
  "gene_symbol": "HIP1",
  "gene_name": "Huntingtin-interacting protein 1",
  "term_label": "clathrin coat assembly"
}